{
  "gene_symbol": "DNAH12",
  "term_label": "Unknown biological process",
  "term_id": "UNKNOWN:0002",
  "gene": "UniProtKB:Q6ZR08",
  "gene_name": "Dynein axonemal heavy chain 12"
}